{
  "gene": "UniProtKB:Q8WWF6",
  "term_label": "Unknown molecular function",
  "gene_name": "DnaJ homolog subfamily B member 3",
  "term_id": "UNKNOWN:0001",
  "gene_symbol": "DNAJB3"
}